{
  "gene": "UniProtKB:Q9NZC9",
  "term_label": "replication fork processing",
  "term_id": "GO:0031297",
  "gene_symbol": "SMARCAL1",
  "gene_name": "SWI_SNF-related matrix-associated actin-dependent regulator of chromatin subfamily A-like protein 1"
}